{
  "gene_symbol": "UQCC3",
  "gene": "UniProtKB:Q6UW78",
  "gene_name": "Ubiquinol-cytochrome-c reductase complex assembly factor 3",
  "term_label": "mitochondrial respiratory chain complex III assembly",
  "term_id": "GO:0034551"
}